GTP-dependent polydeoxyribonucleotide 5'-hydroxyl-kinase activity [GO:0051737] (molecular function) Definition: Catalysis of the reaction: GTP + 5'-dephospho-DNA = GDP + 5'-phospho-DNA. Also known as: GTP-dependent DNA 5'-hydroxyl-kinase activity, GTP-dependent DNA kinase activity, GTP-dependent polydeoxyribonucleotide kinase activity Relationships: is a type of GO:0051735 References: PMID:8428918